{
  "term_id": "GO:0005737",
  "gene_name": "Cannabinoid receptor 1",
  "term_label": "cytoplasm",
  "gene_symbol": "CNR1",
  "gene": "UniProtKB:P21554"
}